{
  "gene": "UniProtKB:Q6UWI4",
  "gene_symbol": "SHISA2",
  "gene_name": "Protein shisa-2 homolog",
  "term_id": "UNKNOWN:0001",
  "term_label": "Unknown molecular function"
}